{
  "term_id": "GO:0042981",
  "gene": "UniProtKB:C9J2P7",
  "gene_symbol": "USP17L15",
  "term_label": "regulation of apoptotic process",
  "gene_name": "Ubiquitin carboxyl-terminal hydrolase 17-like protein 15"
}